chylomicron remnant [GO:0034360] (cellular component) Relationships: is a type of chylomicron [GO:0042627] Definition: A lipoprotein particle that is derived from a mature chylomicron particle by the removal of triglycerides from the chylomicron core by lipoprotein lipase and the subsequent loss of surface components. It characteristically contains apolipoprotein E (APOE) and is cleared from the blood by the liver. Sources: GOC:BHF, GOC:expert_pt, GOC:mah, GOC:rl